androgen binding [GO:0005497] (molecular function) Relationships: is a type of GO:0042562 Definition: Binding to an androgen, a male sex hormone. Sources: GOC:jl